{
  "term_id": "GO:0003950",
  "term_label": "NAD+ poly-ADP-ribosyltransferase activity",
  "gene": "UniProtKB:Q460N5",
  "gene_symbol": "PARP14",
  "gene_name": "Protein mono-ADP-ribosyltransferase PARP14"
}